{
  "gene": "UniProtKB:Q9Y680",
  "term_label": "Unknown cellular component",
  "gene_symbol": "FKBP7",
  "gene_name": "Peptidyl-prolyl cis-trans isomerase FKBP7",
  "term_id": "UNKNOWN:0003"
}